{
  "term_label": "ubiquitin-protein transferase activity",
  "term_id": "GO:0004842",
  "gene_name": "E3 ubiquitin-protein ligase RNF168",
  "gene_symbol": "RNF168",
  "gene": "UniProtKB:Q8IYW5"
}